response to starvation [GO:0042594] (biological process) Relationships: is a type of response to stress [GO:0006950]; is a type of GO:0031667 Definition: Any process that results in a change in state or activity of a cell or an organism (in terms of movement, secretion, enzyme production, gene expression, etc.) as a result of a starvation stimulus, deprivation of nourishment. Sources: GOC:go_curators Subtypes: cellular response to starvation [GO:0009267], GO:0030583, filamentous growth of a population of unicellular organisms in response to starvation [GO:0036170], behavioral response to starvation [GO:0042595], response to nitrate starvation [GO:0090548], response to carbon starvation [GO:0090549], response to molybdenum starvation [GO:0090550], programmed necrotic cell death in response to starvation [GO:0097385], response to metal ion starvation [GO:0180055], GO:1990928